alpha-thujene synthase activity [GO:0102700] (molecular function) Relationships: is a type of carbon-oxygen lyase activity, acting on phosphates [GO:0016838] Sources: MetaCyc:RXN-5105 Definition: Catalysis of the reaction: geranyl diphosphate(3-) = alpha-thujene + diphosphoric acid.